{
  "term_id": "GO:0005615",
  "term_label": "extracellular space",
  "gene_name": "Proteoglycan 4",
  "gene_symbol": "PRG4",
  "gene": "UniProtKB:Q92954"
}